{
  "gene_name": "G-protein coupled receptor 84",
  "gene": "UniProtKB:Q9NQS5",
  "term_label": "urotensin II receptor activity",
  "gene_symbol": "GPR84",
  "term_id": "GO:0001604"
}